{
  "gene_name": "RNA-binding protein 24",
  "term_id": "GO:0010831",
  "gene": "UniProtKB:Q9BX46",
  "term_label": "positive regulation of myotube differentiation",
  "gene_symbol": "RBM24"
}